phloem development [GO:0010088] (biological process) Definition: The formation of the principal food-conducting tissue of a vascular plant. Sources: GOC:tb, ISBN:0471245208 Also known as: phloem histogenesis Relationships: is a type of phloem or xylem histogenesis [GO:0010087]